{
  "gene": "UniProtKB:Q96M85",
  "gene_symbol": "Q96M85",
  "gene_name": "Putative uncharacterized protein FLJ32756",
  "term_label": "Unknown molecular function",
  "term_id": "UNKNOWN:0001"
}